{
  "gene_symbol": "DOP1B",
  "gene_name": "Protein dopey-2",
  "gene": "UniProtKB:Q9Y3R5",
  "term_id": "UNKNOWN:0001",
  "term_label": "Unknown molecular function"
}